methyltetrahydrofolate:corrinoid/iron-sulfur protein methyltransferase activity [GO:0102036] (molecular function) Relationships: is a type of GO:0008168 References: PMID:7928975 Sources: EC:2.1.1.258, GOC:pz Definition: Catalysis of the reaction: a tetrahydrofolate + a [methyl-Co(III) corrinoid Fe-S protein] = an N5-methyl-tetrahydrofolate + a [Co(I) corrinoid Fe-S protein].